terpentetriene synthase activity [GO:0052679] (molecular function) Also known as: terpentedienyl-diphosphate diphosphate-lyase (terpentetriene-forming) activity Sources: RHEA:25617 Relationships: is a type of carbon-oxygen lyase activity, acting on phosphates [GO:0016838] Definition: Catalysis of the reaction: terpentedienyl diphosphate = diphosphate + terpentetriene.